mitochondrial threonyl-tRNA aminoacylation [GO:0070159] (biological process) Relationships: is a type of threonyl-tRNA aminoacylation [GO:0006435]; is a type of GO:0070127 Sources: GOC:mah, GOC:mcc Definition: The process of coupling threonine to threonyl-tRNA in a mitochondrion, catalyzed by threonyl-tRNA synthetase. In tRNA aminoacylation, the amino acid is first activated by linkage to AMP and then transferred to either the 2'- or the 3'-hydroxyl group of the 3'-adenosine residue of the tRNA.